cytosolic small ribosomal subunit [GO:0022627] (cellular component) Relationships: is a type of small ribosomal subunit [GO:0015935]; is part of GO:0022626 Also known as: 30S ribosomal subunit, 40S ribosomal subunit, eukaryotic ribosomal SSU, prokaryotic small ribosomal subunit Sources: GOC:mtg_sensu Definition: The small subunit of a ribosome located in the cytosol.